{
  "gene_name": "NEDD4 family-interacting protein 1",
  "term_id": "GO:0048471",
  "term_label": "perinuclear region of cytoplasm",
  "gene": "UniProtKB:Q9BT67",
  "gene_symbol": "NDFIP1"
}